{
  "gene_name": "Guanine nucleotide-binding protein G(s) subunit alpha isoforms XLas",
  "term_label": "G-protein beta/gamma-subunit complex binding",
  "gene_symbol": "GNAS",
  "gene": "UniProtKB:Q5JWF2",
  "term_id": "GO:0031683"
}